{
  "gene_name": "Dynein axonemal assembly factor 8",
  "gene": "UniProtKB:Q8IYS4",
  "term_label": "dynein axonemal particle",
  "gene_symbol": "DNAAF8",
  "term_id": "GO:0120293"
}